{
  "gene_name": "Spindlin-2B",
  "gene": "UniProtKB:Q9BPZ2",
  "term_id": "GO:0005829",
  "term_label": "cytosol",
  "gene_symbol": "SPIN2B"
}